guanine binding [GO:0002057] (molecular function) Definition: Binding to guanine. Sources: GOC:hjd Relationships: is a type of GO:0002060